{
  "gene_symbol": "C4BPB",
  "gene_name": "C4b-binding protein beta chain",
  "term_label": "Unknown biological process",
  "term_id": "UNKNOWN:0002",
  "gene": "UniProtKB:P20851"
}